nicotinamide riboside transport [GO:0034258] (biological process) Sources: GOC:se Relationships: is a type of nucleoside transport [GO:0015858] Definition: The directed movement of a nicotinamide riboside, which is a pyridine-3-carboxamide covalently bonded to a ribose sugar, into, out of or within a cell, or between cells, by means of some agent such as a transporter or pore.